{
  "term_id": "GO:0043235",
  "term_label": "receptor complex",
  "gene_name": "BTB_POZ domain-containing protein KCTD12",
  "gene": "UniProtKB:Q96CX2",
  "gene_symbol": "KCTD12"
}